{
  "gene_name": "Rho GTPase-activating protein 44",
  "gene": "UniProtKB:Q17R89",
  "term_label": "presynaptic active zone",
  "term_id": "GO:0048786",
  "gene_symbol": "ARHGAP44"
}